{
  "gene_name": "Protein spinster homolog 1",
  "term_label": "transmembrane transporter activity",
  "term_id": "GO:0022857",
  "gene": "UniProtKB:Q9H2V7",
  "gene_symbol": "SPNS1"
}